positive regulation of lymphocyte migration [GO:2000403] (biological process) Subtypes: positive regulation of lymphocyte chemotaxis [GO:0140131], positive regulation of T cell migration [GO:2000406] Sources: GOC:mah Relationships: is a type of positive regulation of mononuclear cell migration [GO:0071677]; is a type of regulation of lymphocyte migration [GO:2000401]; positively regulates GO:0072676 Definition: Any process that activates or increases the frequency, rate or extent of lymphocyte migration.